RNA polymerase III general transcription initiation factor binding [GO:0001025] (molecular function) Sources: GOC:txnOH Subtypes: GO:0001154, TFIIIA-class transcription factor binding [GO:0001155], TFIIIC-class transcription factor complex binding [GO:0001156] Also known as: RNA polymerase III transcription factor binding Relationships: is a type of general transcription initiation factor binding [GO:0140296] Definition: Binding to an RNA polymerase III transcription factor, a protein required to initiate or regulate transcription by RNA polymerase III.